4-hydroxytryptamine 4-phosphate methyltransferase activity [GO:0140381] (molecular function) Also known as: norbaeocystin methyltransferase, psilocybin synthase References: PMID:28763571 Definition: Catalysis of the reaction: 2 S-adenosyl-L-methionine (SAM) + 4-hydroxytryptamine 4-phosphate (norbaeocystin) = 2 S-adenosyl-L-homocysteine + psilocybin. Relationships: is a type of methyltransferase activity [GO:0008168]